enterobacterial common antigen metabolic process [GO:0046378] (biological process) Definition: The chemical reactions and pathways involving enterobacterial common antigen, an acidic polysaccharide containing N-acetyl-D-glucosamine, N-acetyl-D-mannosaminouronic acid, and 4-acetamido-4,6-dideoxy-D-galactose. A major component of the cell wall outer membrane of Gram-negative bacteria. Also known as: enterobacterial common antigen metabolism Sources: GOC:ma Relationships: is_a polysaccharide metabolic process [GO:0005976]; is a type of carbohydrate derivative metabolic process [GO:1901135] Subtypes: enterobacterial common antigen biosynthetic process [GO:0009246]